{
  "gene_name": "Signal-induced proliferation-associated 1-like protein 1",
  "gene": "UniProtKB:O43166",
  "term_id": "GO:0048167",
  "term_label": "regulation of synaptic plasticity",
  "gene_symbol": "SIPA1L1"
}